cellular response to norepinephrine stimulus [GO:0071874] (biological process) Note: Note that epinephrine and norepinephrine are ligands for the same receptors, and there are multiple adrenergic receptors. Relationships: is a type of cellular response to catecholamine stimulus [GO:0071870]; is a type of response to norepinephrine [GO:0071873] Definition: Any process that results in a change in state or activity of a cell (in terms of movement, secretion, enzyme production, gene expression, etc.) as a result of a norepinephrine stimulus. Norepinephrine is a catecholamine that has the formula C8H11NO3; it acts as a hormone, and as a neurotransmitter in most of the sympathetic nervous system. Sources: GOC:BHF, GOC:mah Also known as: cellular response to noradrenaline stimulus